{
  "gene_name": "Equatorin",
  "term_id": "GO:0007342",
  "term_label": "fusion of sperm to egg plasma membrane involved in single fertilization",
  "gene": "UniProtKB:Q9NQ60",
  "gene_symbol": "EQTN"
}